{
  "gene": "UniProtKB:O00483",
  "term_id": "UNKNOWN:0002",
  "gene_name": "Cytochrome c oxidase subunit NDUFA4",
  "term_label": "Unknown biological process",
  "gene_symbol": "NDUFA4"
}